{
  "gene": "UniProtKB:Q9UF56",
  "term_id": "UNKNOWN:0001",
  "term_label": "Unknown molecular function",
  "gene_name": "F-box_LRR-repeat protein 17",
  "gene_symbol": "FBXL17"
}